T cell proliferation involved in immune response [GO:0002309] (biological process) Relationships: is a type of GO:0002286; is a type of GO:0042098 Also known as: T cell proliferation during immune response, T lymphocyte proliferation during immune response, T-cell proliferation during immune response, T-lymphocyte proliferation during immune response Definition: The expansion of a T cell population by cell division as part of an immune response. Sources: GOC:add, ISBN:0781735149 Subtypes: alpha-beta T cell proliferation involved in immune response [GO:0002310], gamma-delta T cell proliferation involved in immune response [GO:0002311]